{
  "term_id": "GO:0009986",
  "gene_name": "Receptor activity-modifying protein 1",
  "gene_symbol": "RAMP1",
  "gene": "UniProtKB:O60894",
  "term_label": "cell surface"
}